cytokine precursor processing [GO:0140447] (biological process) Relationships: is a type of signaling receptor ligand precursor processing [GO:0140448]; is part of cytokine production [GO:0001816] References: PMID:29247995 Definition: The cleavage of a peptide bond in a precursor form of a cytokine, resulting in the mature (active) form of the cytokine. Also known as: interleukin maturation, interleukin processing